cap-independent translational initiation [GO:0002190] (biological process) Subtypes: cap-independent translational initiation of linear mRNA [GO:0110017], cap-independent translational initiation of circular RNA [GO:0110018] References: PMID:17284590 Definition: The process where translation initiation recruits the 40S ribosomal subunits in a Cap and 5' end independent fashion before an AUG codon is encountered in an appropriate sequence context to initiate mRNA or circRNA translation. Regulation: regulated by GO:1903677; negatively regulated by negative regulation of cap-independent translational initiation [GO:1903678]; RO_0002213 by positive regulation of cap-independent translational initiation [GO:1903679] Relationships: is a type of cytoplasmic translational initiation [GO:0002183]